fused antrum stage [GO:0048165] (biological process) Also known as: mammalian oogenesis stage 8 Definition: The stage in oogenesis when the antral spaces fuse to form a single antral space. The oocyte is suspended in the cumulus oophorous and the first polar body in the perivitelline space. Relationships: is a type of mammalian oogenesis stage [GO:0022605] Sources: GOC:jid, GOC:mtg_sensu, ISBN:0198542771